{
  "gene": "UniProtKB:O43280",
  "term_label": "alpha,alpha-trehalase activity",
  "gene_symbol": "TREH",
  "gene_name": "Trehalase",
  "term_id": "GO:0004555"
}